SOD1-calcineurin complex [GO:0032517] (cellular component) Definition: A protein complex formed by the association of superoxide dismutase 1 (SOD1) with calcineurin; complex formation is implicated in activation of calcineurin by SOD1. References: PMID:17324120 Sources: GOC:mah Relationships: is_a intracellular protein-containing complex [GO:0140535]